{
  "gene_name": "Protein YIF1A",
  "gene": "UniProtKB:O95070",
  "term_id": "GO:0005789",
  "gene_symbol": "YIF1A",
  "term_label": "endoplasmic reticulum membrane"
}